MyD88-dependent toll-like receptor 4 signaling pathway [GO:0035660] (biological process) Relationships: is a type of MyD88-dependent toll-like receptor signaling pathway [GO:0002755]; is a type of toll-like receptor 4 signaling pathway [GO:0034142] Definition: The series of molecular signals initiated by a ligand binding to a toll-like 4 receptor, where the MyD88 adaptor molecule mediates transduction of the signal. Toll-like 4 receptors bind bacterial lipopolysaccharide (LPS) to initiate an innate immune response. References: PMID:18304834, PMID:20385024 Sources: GOC:BHF Also known as: MyD88-dependent TLR4 signaling pathway, MyD88-dependent toll-like receptor 4 signalling pathway